{
  "term_id": "UNKNOWN:0002",
  "term_label": "Unknown biological process",
  "gene_name": "Putative uncharacterized protein FLJ92257",
  "gene": "UniProtKB:Q75L30",
  "gene_symbol": "Q75L30"
}